negative regulation of reactive oxygen species metabolic process [GO:2000378] (biological process) Definition: Any process that stops, prevents or reduces the frequency, rate or extent of reactive oxygen species metabolic process. Subtypes: GO:0010727, GO:0032929, negative regulation of reactive oxygen species biosynthetic process [GO:1903427], negative regulation of removal of superoxide radicals [GO:1904832] Sources: GOC:mah Relationships: is a type of negative regulation of metabolic process [GO:0009892]; is_a regulation of reactive oxygen species metabolic process [GO:2000377]; negatively regulates reactive oxygen species metabolic process [GO:0072593] Also known as: negative regulation of ROS metabolic process, negative regulation of reactive oxygen species metabolism